regulation of monoatomic cation transmembrane transport [GO:1904062] (biological process) Definition: Any process that modulates the frequency, rate or extent of cation transmembrane transport. References: PMID:15304482 Sources: GOC:TermGenie, GO_REF:0000058 Also known as: regulation of cation transmembrane transport Subtypes: regulation of proton transport [GO:0010155], regulation of iron ion transmembrane transport [GO:0034759], regulation of zinc ion transmembrane transport [GO:0071580], GO:1901379, regulation of sodium ion transmembrane transport [GO:1902305], regulation of copper ion transmembrane transport [GO:1902311], regulation of calcium ion transmembrane transport [GO:1903169], GO:1904063, GO:1904064 Relationships: is a type of GO:0034765; RO_0002211 monoatomic cation transmembrane transport [GO:0098655]